{
  "term_label": "Unknown biological process",
  "gene_name": "G2 and S phase-expressed protein 1",
  "gene": "UniProtKB:Q9NYZ3",
  "gene_symbol": "GTSE1",
  "term_id": "UNKNOWN:0002"
}